{
  "term_label": "carboxylesterase activity",
  "gene_symbol": "CES1P1",
  "term_id": "GO:0106435",
  "gene": "UniProtKB:Q9UKY3",
  "gene_name": "Putative inactive carboxylesterase 4"
}